negative regulation of outer hair cell apoptotic process [GO:1905586] (biological process) References: PMID:24472721 Sources: GOC:TermGenie, GO_REF:0000058 Relationships: is a type of negative regulation of neuron apoptotic process [GO:0043524]; is a type of regulation of outer hair cell apoptotic process [GO:1905585]; negatively regulates outer hair cell apoptotic process [GO:1905584] Also known as: down regulation of cochlear outer hair cell apoptotic process, down regulation of outer hair cell apoptotic process, down-regulation of cochlear outer hair cell apoptotic process, down-regulation of outer hair cell apoptotic process, downregulation of cochlear outer hair cell apoptotic process, downregulation of outer hair cell apoptotic process, negative regulation of cochlear outer hair cell apoptotic process, down regulation of cochlear outer hair cell apoptosis, down regulation of outer hair cell apoptosis, down-regulation of cochlear outer hair cell apoptosis, down-regulation of outer hair cell apoptosis, downregulation of cochlear outer hair cell apoptosis, downregulation of outer hair cell apoptosis, inhibition of cochlear outer hair cell apoptosis, inhibition of cochlear outer hair cell apoptotic process, inhibition of outer hair cell apoptosis, inhibition of outer hair cell apoptotic process, negative regulation of cochlear outer hair cell apoptosis, negative regulation of outer hair cell apoptosis Definition: Any process that stops, prevents or reduces the frequency, rate or extent of outer hair cell apoptotic process.